{
  "gene_symbol": "CHCHD2",
  "term_label": "mitochondrion",
  "gene": "UniProtKB:Q9Y6H1",
  "term_id": "GO:0005739",
  "gene_name": "Coiled-coil-helix-coiled-coil-helix domain-containing protein 2"
}